{
  "gene_name": "Histone H4 transcription factor",
  "gene_symbol": "HINFP",
  "term_id": "GO:0000978",
  "term_label": "RNA polymerase II cis-regulatory region sequence-specific DNA binding",
  "gene": "UniProtKB:Q9BQA5"
}